{
  "term_label": "mitochondrial respiratory chain complex IV assembly",
  "term_id": "GO:0033617",
  "gene_name": "Small integral membrane protein 20",
  "gene": "UniProtKB:Q8N5G0",
  "gene_symbol": "SMIM20"
}